{
  "gene": "UniProtKB:Q9UJW7",
  "term_label": "regulation of transcription by RNA polymerase II",
  "term_id": "GO:0006357",
  "gene_symbol": "ZNF229",
  "gene_name": "Zinc finger protein 229"
}